{
  "gene": "UniProtKB:Q01546",
  "term_id": "GO:0030280",
  "gene_name": "Keratin, type II cytoskeletal 2 oral",
  "term_label": "structural constituent of skin epidermis",
  "gene_symbol": "KRT76"
}